{
  "gene_symbol": "GAGE8",
  "gene_name": "G antigen 2D",
  "term_id": "UNKNOWN:0002",
  "term_label": "Unknown biological process",
  "gene": "UniProtKB:Q9UEU5"
}